{
  "gene_symbol": "BTNL2",
  "term_id": "GO:0005102",
  "gene_name": "Butyrophilin-like protein 2",
  "gene": "UniProtKB:Q9UIR0",
  "term_label": "signaling receptor binding"
}